astral microtubule [GO:0000235] (cellular component) Definition: Any of the spindle microtubules that radiate in all directions from the spindle poles and are thought to contribute to the forces that separate the poles and position them in relation to the rest of the cell. Subtypes: mitotic spindle astral microtubule [GO:0061673], GO:1990574 Sources: ISBN:0815316194 Relationships: is a type of spindle microtubule [GO:0005876]; is a type of cytoplasmic microtubule [GO:0005881]; is part of aster [GO:0005818]